cardiac vascular smooth muscle cell differentiation [GO:0060947] (biological process) Sources: GOC:mtg_heart Also known as: heart vascular smooth muscle cell differentiation Subtypes: epicardium-derived cardiac vascular smooth muscle cell differentiation [GO:0060983] Regulation: regulated by regulation of cardiac vascular smooth muscle cell differentiation [GO:2000722]; RO_0002212 by negative regulation of cardiac vascular smooth muscle cell differentiation [GO:2000723]; positively regulated by GO:2000724 Relationships: is a type of GO:0035051; is a type of vascular associated smooth muscle cell differentiation [GO:0035886]; is part of coronary vasculature development [GO:0060976] Definition: The process in which a relatively unspecialized cell acquires specialized features of a cardiac vascular smooth muscle cell. A cardiac vascular smooth muscle cell covers the heart vasculature and lacks transverse striations in its constituent fibers.